{
  "term_id": "GO:0006122",
  "gene_name": "Cytochrome c",
  "gene_symbol": "CYCS",
  "gene": "UniProtKB:P99999",
  "term_label": "mitochondrial electron transport, ubiquinol to cytochrome c"
}